{
  "gene_name": "Centrosomal AT-AC splicing factor",
  "gene_symbol": "CENATAC",
  "term_id": "UNKNOWN:0001",
  "term_label": "Unknown molecular function",
  "gene": "UniProtKB:Q86UT8"
}